positive regulation of mRNA cis splicing, via spliceosome [GO:1905746] (biological process) Relationships: is a type of positive regulation of mRNA splicing, via spliceosome [GO:0048026]; is a type of regulation of mRNA cis splicing, via spliceosome [GO:1905744]; positively regulates mRNA cis splicing, via spliceosome [GO:0045292] References: PMID:2880558 Sources: GOC:TermGenie, GO_REF:0000058 Definition: Any process that activates or increases the frequency, rate or extent of mRNA cis splicing, via spliceosome.